{
  "gene_symbol": "ALCAM",
  "term_id": "GO:0007155",
  "gene": "UniProtKB:Q13740",
  "term_label": "cell adhesion",
  "gene_name": "CD166 antigen"
}